{
  "gene_symbol": "ANXA11",
  "term_label": "phagocytosis",
  "gene": "UniProtKB:P50995",
  "gene_name": "Annexin A11",
  "term_id": "GO:0006909"
}